proteoglycan biosynthetic process [GO:0030166] (biological process) Definition: The chemical reactions and pathways resulting in the formation of proteoglycans, any glycoprotein in which the carbohydrate units are glycosaminoglycans. Also known as: proteoglycan anabolism, proteoglycan biosynthesis, proteoglycan formation, proteoglycan synthesis Regulation: negatively regulated by GO:1902729; positively regulated by positive regulation of proteoglycan biosynthetic process [GO:1902730] References: PMID:35536939 Subtypes: heparan sulfate proteoglycan biosynthetic process [GO:0015012], keratan sulfate proteoglycan biosynthetic process [GO:0018146], chondroitin sulfate proteoglycan biosynthetic process [GO:0050650], GO:0050651 Relationships: is a type of proteoglycan metabolic process [GO:0006029]; is_a glycoprotein biosynthetic process [GO:0009101]